{
  "term_id": "GO:0030198",
  "gene": "UniProtKB:A6NHS7",
  "gene_name": "MANSC domain-containing protein 4",
  "gene_symbol": "MANSC4",
  "term_label": "extracellular matrix organization"
}